{
  "gene_name": "BCAS3 microtubule associated cell migration factor",
  "term_label": "Unknown molecular function",
  "gene": "UniProtKB:Q9H6U6",
  "term_id": "UNKNOWN:0001",
  "gene_symbol": "BCAS3"
}